natural killer cell mediated cytotoxicity directed against tumor cell target [GO:0002420] (BP) Definition: The directed killing of a tumor cell by a natural killer cell through the release of granules containing cytotoxic mediators or through the engagement of death receptors. References: PMID:16730260 Sources: GOC:add, ISBN:0781735149 Also known as: NK cell mediated cytotoxicity directed against tumor cell target Note: Note that either or both mechanisms mentioned in the definition may be used in this process. Note that both granule release and the engagement of death receptors on target cells result in induction of apoptosis in the target cell. Relationships: is a type of natural killer cell mediated immune response to tumor cell [GO:0002423]; is a type of natural killer cell mediated cytotoxicity [GO:0042267] Regulation: regulated by regulation of natural killer cell mediated cytotoxicity directed against tumor cell target [GO:0002858]; negatively regulated by GO:0002859; positively regulated by GO:0002860